{
  "gene": "UniProtKB:Q96C19",
  "gene_symbol": "EFHD2",
  "term_id": "GO:0005509",
  "gene_name": "EF-hand domain-containing protein D2",
  "term_label": "calcium ion binding"
}